{
  "gene_symbol": "CCDC70",
  "gene": "UniProtKB:Q6NSX1",
  "term_label": "Unknown molecular function",
  "gene_name": "Coiled-coil domain-containing protein 70",
  "term_id": "UNKNOWN:0001"
}